{
  "gene": "UniProtKB:Q4KMZ1",
  "term_label": "Unknown molecular function",
  "gene_symbol": "IQCC",
  "term_id": "UNKNOWN:0001",
  "gene_name": "IQ domain-containing protein C"
}